{
  "gene_symbol": "CFI",
  "gene_name": "Complement factor I",
  "gene": "UniProtKB:P05156",
  "term_label": "serine-type peptidase activity",
  "term_id": "GO:0008236"
}